L-tyrosine-pyruvate transaminase activity [GO:0080098] (molecular function) Definition: Catalysis of the reaction: L-tyrosine + pyruvate = (4-hydroxyphenyl)pyruvate + L-alanine. Sources: MetaCyc:RXN3O-4157 Relationships: is_a aromatic-amino-acid transaminase activity [GO:0008793] Also known as: L-tyrosine aminotransferase activity, L-tyrosine:pyruvate aminotransferase activity